{
  "gene_name": "Heparan-sulfate 6-O-sulfotransferase 3",
  "gene": "UniProtKB:Q8IZP7",
  "term_label": "heparan sulfate proteoglycan biosynthetic process",
  "term_id": "GO:0015012",
  "gene_symbol": "HS6ST3"
}